{
  "term_id": "GO:0048240",
  "gene_name": "Semenogelin-2",
  "gene": "UniProtKB:Q02383",
  "gene_symbol": "SEMG2",
  "term_label": "sperm capacitation"
}